{
  "term_id": "GO:0071385",
  "term_label": "cellular response to glucocorticoid stimulus",
  "gene_name": "UDP-glucuronosyltransferase 1A9",
  "gene": "UniProtKB:O60656",
  "gene_symbol": "UGT1A9"
}